low-affinity IgM receptor activity [GO:0002173] (molecular function) Relationships: is a type of IgM receptor activity [GO:0001793] Definition: Combining with low affinity with an immunoglobulin of an IgM isotype via the Fc region, and transmitting the signal from one side of the membrane to the other to initiate a change in cell activity. Also known as: low affinity IgM receptor activity Sources: GOC:hjd, GOC:signaling